{
  "gene_symbol": "CHRM4",
  "gene": "UniProtKB:P08173",
  "gene_name": "Muscarinic acetylcholine receptor M4",
  "term_label": "plasma membrane",
  "term_id": "GO:0005886"
}